{
  "gene": "UniProtKB:P32519",
  "term_id": "GO:0005634",
  "gene_name": "ETS-related transcription factor Elf-1",
  "term_label": "nucleus",
  "gene_symbol": "ELF1"
}